plasma membrane bounded cell projection cytoplasm [GO:0032838] (cellular component) Relationships: is a type of cytoplasmic region [GO:0099568]; is part of plasma membrane bounded cell projection [GO:0120025] Definition: All of the contents of a plasma membrane bounded cell projection, excluding the plasma membrane surrounding the projection. Subtypes: ciliary plasm [GO:0097014], GO:0120111 Sources: GOC:krc, GOC:mah